{
  "gene": "UniProtKB:Q99456",
  "term_label": "intermediate filament organization",
  "gene_name": "Keratin, type I cytoskeletal 12",
  "gene_symbol": "KRT12",
  "term_id": "GO:0045109"
}